regulation of motor neuron axon guidance [GO:1905812] (biological process) References: PMID:18434533 Sources: GOC:TermGenie, GO_REF:0000058 Subtypes: negative regulation of motor neuron axon guidance [GO:1905813], positive regulation of motor neuron axon guidance [GO:1905814] Also known as: regulation of motoneuron axon guidance, regulation of motor axon guidance, regulation of motor axon pathfinding Relationships: is a type of GO:1902667; regulates motor neuron axon guidance [GO:0008045] Definition: Any process that modulates the frequency, rate or extent of motor neuron axon guidance.